{
  "gene": "UniProtKB:Q15546",
  "gene_symbol": "MMD",
  "term_id": "UNKNOWN:0001",
  "term_label": "Unknown molecular function",
  "gene_name": "Monocyte to macrophage differentiation factor"
}